positive regulation of maintenance of mitotic sister chromatid cohesion, telomeric [GO:1904909] (biological process) Also known as: positive regulation of maintenance of mitotic sister chromatin cohesion at telomere, positive regulation of maintenance of sister chromatin cohesion at telomere at mitosis, positive regulation of maintenance of telomeric mitotic sister chromatin cohesion, up regulation of maintenance of mitotic sister chromatid cohesion, telomeric, up regulation of maintenance of mitotic sister chromatin cohesion at telomere, up regulation of maintenance of sister chromatin cohesion at telomere at mitosis, up regulation of maintenance of telomeric mitotic sister chromatin cohesion, up-regulation of maintenance of mitotic sister chromatid cohesion, telomeric, up-regulation of maintenance of mitotic sister chromatin cohesion at telomere, up-regulation of maintenance of sister chromatin cohesion at telomere at mitosis, up-regulation of maintenance of telomeric mitotic sister chromatin cohesion, upregulation of maintenance of mitotic sister chromatid cohesion, telomeric, upregulation of maintenance of mitotic sister chromatin cohesion at telomere, upregulation of maintenance of sister chromatin cohesion at telomere at mitosis, upregulation of maintenance of telomeric mitotic sister chromatin cohesion, activation of maintenance of mitotic sister chromatid cohesion, telomeric, activation of maintenance of mitotic sister chromatin cohesion at telomere, activation of maintenance of sister chromatin cohesion at telomere at mitosis, activation of maintenance of telomeric mitotic sister chromatin cohesion References: PMID:26373281 Sources: GOC:BHF, GOC:BHF_telomere, GOC:TermGenie, GOC:rph, GO_REF:0000058 Relationships: is a type of positive regulation of maintenance of mitotic sister chromatid cohesion [GO:0034184]; is a type of regulation of maintenance of mitotic sister chromatid cohesion, telomeric [GO:1904907]; positively regulates maintenance of mitotic sister chromatid cohesion, telomeric [GO:0099403] Definition: Any process that activates or increases the frequency, rate or extent of maintenance of mitotic sister chromatid cohesion, telomeric.